regulation of mast cell activation [GO:0033003] (biological process) Definition: Any process that modulates the frequency, rate, or extent of mast cell activation. Subtypes: GO:0033004, positive regulation of mast cell activation [GO:0033005], regulation of mast cell activation involved in immune response [GO:0033006] Sources: GOC:mah Relationships: is a type of regulation of leukocyte activation [GO:0002694]; regulates mast cell activation [GO:0045576]